{
  "gene": "UniProtKB:Q8TDY2",
  "gene_symbol": "RB1CC1",
  "term_id": "GO:0034517",
  "term_label": "ribophagy",
  "gene_name": "RB1-inducible coiled-coil protein 1"
}